regulation of (1->3)-alpha-glucan biosynthetic process [GO:0070606] (biological process) Relationships: is a type of regulation of alpha-glucan biosynthetic process [GO:0032949]; regulates (1->3)-alpha-glucan biosynthetic process [GO:0070596] Definition: Any process that modulates the frequency, rate or extent of the chemical reactions and pathways resulting in the formation of (1->3)-alpha-D-glucans, compounds composed of glucose residues linked by (1->3)-alpha-D-glucosidic bonds. Also known as: regulation of 1,3-alpha-glucan anabolism, regulation of 1,3-alpha-glucan biosynthesis, regulation of 1,3-alpha-glucan biosynthetic process, regulation of 1,3-alpha-glucan formation, regulation of 1,3-alpha-glucan synthesis, regulation of alpha-1,3 glucan anabolism, regulation of alpha-1,3 glucan biosynthesis, regulation of alpha-1,3 glucan biosynthetic process, regulation of alpha-1,3 glucan formation, regulation of alpha-1,3 glucan synthesis Sources: GOC:mah Subtypes: GO:0070608